{
  "gene_symbol": "AGBL1",
  "term_id": "UNKNOWN:0002",
  "gene": "UniProtKB:Q96MI9",
  "gene_name": "Cytosolic carboxypeptidase 4",
  "term_label": "Unknown biological process"
}